{
  "term_id": "GO:0009897",
  "term_label": "external side of plasma membrane",
  "gene_symbol": "CLEC4A",
  "gene": "UniProtKB:Q9UMR7",
  "gene_name": "C-type lectin domain family 4 member A"
}